twitch skeletal muscle contraction [GO:0014721] (BP) Definition: A process in which force is generated within twitch skeletal muscle tissue, resulting in a change in muscle geometry. Force generation involves a chemo-mechanical energy conversion step that is carried out by the actin/myosin complex activity, which generates force through ATP hydrolysis. The twitch skeletal muscle responds to neurostimulations with a contraction followed by a relaxation. Sources: GOC:mtg_muscle Relationships: is a type of GO:0003010 Subtypes: fast-twitch skeletal muscle fiber contraction [GO:0031443], slow-twitch skeletal muscle fiber contraction [GO:0031444] Regulation: regulated by regulation of twitch skeletal muscle contraction [GO:0014724]